{
  "term_id": "GO:0042605",
  "term_label": "peptide antigen binding",
  "gene_name": "HLA class II histocompatibility antigen, DRB1 beta chain",
  "gene": "UniProtKB:P01911",
  "gene_symbol": "HLA-DRB1"
}